{
  "term_id": "GO:0005783",
  "term_label": "endoplasmic reticulum",
  "gene": "UniProtKB:Q15125",
  "gene_name": "3-beta-hydroxysteroid-Delta(8),Delta(7)-isomerase",
  "gene_symbol": "EBP"
}